{
  "term_id": "GO:0070374",
  "gene_name": "Pituitary adenylate cyclase-activating polypeptide",
  "gene_symbol": "ADCYAP1",
  "gene": "UniProtKB:P18509",
  "term_label": "positive regulation of ERK1 and ERK2 cascade"
}